terminal region determination [GO:0007362] (biological process) Relationships: is a type of embryonic pattern specification [GO:0009880]; is part of GO:0007354 Definition: Specification of the terminal regions (the two non-segmented ends) of the embryo by the gap genes; exemplified in insects by the actions of huckebein and tailless gene products. Sources: ISBN:0879694238, http://fly.ebi.ac.uk/allied-data/lk/interactive-fly/aimain/1aahome.htm